ketone catabolic process [GO:0042182] (biological process) Regulation: regulated by regulation of ketone catabolic process [GO:0010567] Also known as: ketone breakdown, ketone catabolism, ketone degradation Definition: The chemical reactions and pathways resulting in the breakdown of ketones, a class of organic compounds that contain the carbonyl group, CO, and in which the carbonyl group is bonded only to carbon atoms. The general formula for a ketone is RCOR, where R and R are alkyl or aryl groups. Relationships: is a type of ketone metabolic process [GO:0042180]; is a type of small molecule catabolic process [GO:0044282] Subtypes: progesterone catabolic process [GO:0006709], adamantanone catabolic process [GO:0019263], (+)-camphor catabolic process [GO:0019383], aldosterone catabolic process [GO:0032343], curcumin catabolic process [GO:0036040], GO:0036183, menaquinone catabolic process [GO:0042361], vitamin K catabolic process [GO:0042377], acetoin catabolic process [GO:0045150], GO:0046213, chalcone catabolic process [GO:0046280], ecdysteroid catabolic process [GO:0046344], methylglyoxal catabolic process [GO:0051596], GO:0062175, GO:0097053, asperfuranone catabolic process [GO:1900553], emodin catabolic process [GO:1900574], endocrocin catabolic process [GO:1900601], tensidol A catabolic process [GO:1900604], GO:1900607, averantin catabolic process [GO:1900762], GO:1900765, GO:1900786, GO:1900792, cspyrone B1 catabolic process [GO:1900801], helvolic acid catabolic process [GO:1900811], monodictyphenone catabolic process [GO:1900814], tetracenomycin C catabolic process [GO:1901105], granaticin catabolic process [GO:1901108], funalenone catabolic process [GO:1901365], quinone catabolic process [GO:1901662], daunorubicin catabolic process [GO:1901770], mitomycin C catabolic process [GO:1901776], 1,5-anhydro-D-fructose catabolic process [GO:1901802], ecgonone methyl ester catabolic process [GO:1901871], neosartoricin catabolic process [GO:1902049], GO:1902382, GO:1902385 Sources: GOC:go_curators